{
  "term_label": "antigen processing and presentation of endogenous peptide antigen via MHC class Ib",
  "gene": "UniProtKB:P25311",
  "term_id": "GO:0002476",
  "gene_symbol": "AZGP1",
  "gene_name": "Zinc-alpha-2-glycoprotein"
}